{
  "term_id": "GO:1902476",
  "gene_name": "Solute carrier family 12 member 5",
  "term_label": "chloride transmembrane transport",
  "gene_symbol": "SLC12A5",
  "gene": "UniProtKB:Q9H2X9"
}